{
  "term_label": "BMP signaling pathway",
  "gene_name": "Anti-Muellerian hormone type-2 receptor",
  "gene_symbol": "AMHR2",
  "gene": "UniProtKB:Q16671",
  "term_id": "GO:0030509"
}